{
  "gene": "UniProtKB:O14802",
  "gene_name": "DNA-directed RNA polymerase III subunit RPC1",
  "term_label": "RNA polymerase III complex",
  "term_id": "GO:0005666",
  "gene_symbol": "POLR3A"
}